{
  "gene": "UniProtKB:Q15654",
  "gene_name": "Thyroid receptor-interacting protein 6",
  "term_label": "Unknown molecular function",
  "term_id": "UNKNOWN:0001",
  "gene_symbol": "TRIP6"
}